{
  "gene": "UniProtKB:P61204",
  "gene_symbol": "ARF3",
  "gene_name": "ADP-ribosylation factor 3",
  "term_id": "GO:0016192",
  "term_label": "vesicle-mediated transport"
}